{
  "term_label": "phagocytic vesicle membrane",
  "term_id": "GO:0030670",
  "gene_symbol": "SLC11A1",
  "gene_name": "Natural resistance-associated macrophage protein 1",
  "gene": "UniProtKB:P49279"
}